pectate disaccharide-lyase activity [GO:0047489] (molecular function) Sources: EC:4.2.2.9 Also known as: (1->4)-alpha-D-galacturonan reducing-end-disaccharide-lyase activity, Exo-PATE activity, Exo-PGL activity, PATE activity, exo-PATE, exo-PGL, exopectate lyase activity, exopectic acid transeliminase activity, exopolygalacturonate lyase activity, exopolygalacturonic acid-trans-eliminase activity, pectate exo-lyase activity Relationships: is a type of carbon-oxygen lyase activity, acting on polysaccharides [GO:0016837] Definition: Catalysis of the reaction: a pectate = a pectate + 4-(4-deoxy-alpha-D-galact-4-enuronosyl)-D-galacturonate. This reaction is the eliminative cleavage of 4-(4-deoxy-alpha-D-galact-4-enuronosyl)-D-galacturonate from the reducing end of pectate, i.e. de-esterified pectin.